{
  "gene": "UniProtKB:Q06055",
  "gene_symbol": "ATP5MC2",
  "term_label": "Unknown molecular function",
  "gene_name": "ATP synthase F(0) complex subunit C2, mitochondrial",
  "term_id": "UNKNOWN:0001"
}